{
  "gene_name": "Putative homeobox protein Meis3-like 2",
  "term_label": "nucleus",
  "term_id": "GO:0005634",
  "gene": "UniProtKB:A8K0S8",
  "gene_symbol": "MEIS3P2"
}